{
  "gene_name": "Four and a half LIM domains protein 5",
  "term_id": "GO:0003713",
  "gene": "UniProtKB:Q5TD97",
  "gene_symbol": "FHL5",
  "term_label": "transcription coactivator activity"
}